{
  "term_id": "GO:0005737",
  "gene": "UniProtKB:P35237",
  "term_label": "cytoplasm",
  "gene_name": "Serpin B6",
  "gene_symbol": "SERPINB6"
}